tubulobulbar complex [GO:0036284] (CC) References: PMID:22510523 Sources: GOC:sl Subtypes: apical tubulobulbar complex [GO:0061828], basal tubulobulbar complex [GO:0061829] Also known as: TBC Definition: Actin-based structures involved in establishing close contact between Sertoli-Sertoli cells or Sertoli-spermatids in the seminiferous tubules of the testes. Relationships: is a type of protein-containing complex [GO:0032991]